{
  "term_id": "UNKNOWN:0003",
  "gene_name": "Serine_arginine repetitive matrix protein 5",
  "gene_symbol": "SRRM5",
  "term_label": "Unknown cellular component",
  "gene": "UniProtKB:B3KS81"
}